{
  "term_id": "GO:0042995",
  "term_label": "cell projection",
  "gene": "UniProtKB:P11277",
  "gene_name": "Spectrin beta chain, erythrocytic",
  "gene_symbol": "SPTB"
}